{
  "gene_name": "Casein kinase I isoform delta",
  "term_id": "GO:0007165",
  "gene": "UniProtKB:P48730",
  "gene_symbol": "CSNK1D",
  "term_label": "signal transduction"
}